D-glycero-D-manno-heptose 7-phosphate metabolic process [GO:2001060] (biological process) Also known as: D-glycero-D-manno-heptose 7-phosphate metabolism Definition: The chemical reactions and pathways involving a D-glycero-D-manno-heptose 7-phosphate. Subtypes: GO:2001061 Relationships: is a type of phosphate-containing compound metabolic process [GO:0006796]; is a type of organophosphate metabolic process [GO:0019637]; is a type of GO:1901135 Sources: GOC:mengo_curators